L-cysteine-S-conjugate N-acetyltransferase activity [GO:0047198] (molecular function) Definition: Catalysis of the reaction: S-substituted L-cysteine + acetyl-CoA = S-substituted N-acetyl-L-cysteine + CoA + H+. Also known as: cysteine-S-conjugate N-acetyltransferase activity, acetyl-CoA:S-substituted L-cysteine N-acetyltransferase activity Sources: EC:2.3.1.80, RHEA:19213 Relationships: is a type of L-amino-acid N-acetyltransferase activity [GO:0140085]